{
  "term_id": "GO:0030073",
  "term_label": "insulin secretion",
  "gene_symbol": "FAM3B",
  "gene_name": "Protein FAM3B",
  "gene": "UniProtKB:P58499"
}